{
  "gene_symbol": "EPO",
  "gene": "UniProtKB:P01588",
  "gene_name": "Erythropoietin",
  "term_label": "cell surface receptor signaling pathway via STAT",
  "term_id": "GO:0097696"
}